{
  "gene": "UniProtKB:O15240",
  "gene_symbol": "VGF",
  "term_label": "hormone activity",
  "term_id": "GO:0005179",
  "gene_name": "Neurosecretory protein VGF"
}